{
  "gene_name": "Cyclin-dependent kinase 6",
  "term_label": "signal transduction",
  "term_id": "GO:0007165",
  "gene": "UniProtKB:Q00534",
  "gene_symbol": "CDK6"
}